{
  "gene_name": "Protein unc-119 homolog A",
  "gene_symbol": "UNC119",
  "term_label": "mitotic cytokinesis",
  "term_id": "GO:0000281",
  "gene": "UniProtKB:Q13432"
}